{
  "gene_symbol": "ZXDB",
  "gene": "UniProtKB:P98169",
  "gene_name": "Zinc finger X-linked protein ZXDB",
  "term_label": "nucleus",
  "term_id": "GO:0005634"
}